{
  "gene_symbol": "GGH",
  "term_id": "GO:0005773",
  "term_label": "vacuole",
  "gene": "UniProtKB:Q92820",
  "gene_name": "Gamma-glutamyl hydrolase"
}